{
  "term_label": "regulation of transcription by RNA polymerase II",
  "term_id": "GO:0006357",
  "gene": "UniProtKB:O60682",
  "gene_symbol": "MSC",
  "gene_name": "Musculin"
}